{
  "gene": "UniProtKB:O94805",
  "gene_symbol": "ACTL6B",
  "term_id": "GO:0007399",
  "term_label": "nervous system development",
  "gene_name": "Actin-like protein 6B"
}